xanthommatin reductase activity [GO:0050399] (molecular function) Relationships: is a type of oxidoreductase activity, acting on the CH-CH group of donors, NAD or NADP as acceptor [GO:0016628] Definition: Catalysis of the reaction: 5,12-dihydroxanthommatin + NAD+ = H+ + NADH + xanthommatin. Sources: EC:1.3.1.41, RHEA:13417 Also known as: 5,12-dihydroxanthommatin:NAD+ oxidoreductase activity